cellular response to acetaldehyde [GO:1905641] (biological process) References: PMID:27687866 Sources: GOC:TermGenie, GO_REF:0000071 Definition: Any process that results in a change in state or activity of a cell (in terms of movement, secretion, enzyme production, gene expression, etc.) as a result of an acetaldehyde stimulus. Relationships: is_a cellular response to aldehyde [GO:0110096]; is_a GO:1905640